positive regulation of relaxation of smooth muscle [GO:1901082] (biological process) Subtypes: positive regulation of uterine smooth muscle relaxation [GO:1900721] Also known as: activation of smooth muscle relaxation, positive regulation of smooth muscle relaxation, up regulation of relaxation of smooth muscle, up regulation of smooth muscle relaxation, up-regulation of relaxation of smooth muscle, up-regulation of smooth muscle relaxation, upregulation of relaxation of smooth muscle, upregulation of smooth muscle relaxation, activation of relaxation of smooth muscle Sources: GOC:TermGenie Definition: Any process that activates or increases the frequency, rate or extent of relaxation of smooth muscle. Relationships: is_a positive regulation of relaxation of muscle [GO:1901079]; is a type of regulation of relaxation of smooth muscle [GO:1901080]; positively regulates relaxation of smooth muscle [GO:0044557]